molybdopterin cofactor catabolic process [GO:0032325] (biological process) Definition: The chemical reactions and pathways resulting in the breakdown of the molybdopterin cofactor (Moco), essential for the catalytic activity of some enzymes, e.g. sulfite oxidase, xanthine dehydrogenase, and aldehyde oxidase. The cofactor consists of a mononuclear molybdenum (Mo-molybdopterin) or tungsten ion (W-molybdopterin) coordinated by one or two molybdopterin ligands. Relationships: is a type of GO:0043545; is a type of organophosphate catabolic process [GO:0046434] Subtypes: Mo-molybdopterin cofactor catabolic process [GO:0032326], W-molybdopterin cofactor catabolic process [GO:0032327] Sources: GOC:mah